{
  "gene_name": "Prostaglandin E2 receptor EP3 subtype",
  "term_id": "GO:0007204",
  "term_label": "positive regulation of cytosolic calcium ion concentration",
  "gene_symbol": "PTGER3",
  "gene": "UniProtKB:P43115"
}